{
  "term_label": "Unknown molecular function",
  "gene_name": "Cilium assembly protein DZIP1L",
  "term_id": "UNKNOWN:0001",
  "gene": "UniProtKB:Q8IYY4",
  "gene_symbol": "DZIP1L"
}